{
  "term_id": "GO:0004197",
  "gene": "UniProtKB:P07711",
  "gene_name": "Procathepsin L",
  "gene_symbol": "CTSL",
  "term_label": "cysteine-type endopeptidase activity"
}